negative regulation of hair follicle development [GO:0051799] (biological process) Also known as: down regulation of hair follicle development, down-regulation of hair follicle development, downregulation of hair follicle development, inhibition of hair follicle development Sources: GOC:ai Subtypes: negative regulation of hair follicle maturation [GO:0048817], GO:0061170 Relationships: is a type of negative regulation of developmental process [GO:0051093]; is a type of negative regulation of multicellular organismal process [GO:0051241]; is a type of regulation of hair follicle development [GO:0051797]; negatively regulates GO:0001942 Definition: Any process that stops, prevents, or reduces the frequency, rate or extent of hair follicle development.